hydrazine dehydrogenase activity [GO:0140287] (molecular function) Definition: Catalysis of the reaction: hydrazine + 4 Fe(III)-[cytochrome c] = N2 + 4 Fe(II)-[cytochrome c] + 4 H+. Sources: RHEA:23232 Relationships: is a type of oxidoreductase activity, acting on other nitrogenous compounds as donors, cytochrome as acceptor [GO:0016662]